{
  "term_id": "GO:0030133",
  "gene_name": "Transmembrane protein 187",
  "term_label": "transport vesicle",
  "gene": "UniProtKB:Q14656",
  "gene_symbol": "TMEM187"
}